regulation of proton transport [GO:0010155] (biological process) Definition: Any process that modulates the frequency, rate or extent of proton transport into, out of or within a cell, or between cells, by means of some agent such as a transporter or pore. Sources: GOC:sm Relationships: is a type of regulation of monoatomic cation transmembrane transport [GO:1904062]; regulates proton transmembrane transport [GO:1902600] Subtypes: regulation of synaptic vesicle lumen acidification [GO:1901546], regulation of potassium:proton exchanging ATPase activity [GO:1904451], regulation of cytochrome-c oxidase activity [GO:1904959]